{
  "term_label": "sodium ion export across plasma membrane",
  "gene_symbol": "ATP1B3",
  "gene_name": "Sodium_potassium-transporting ATPase subunit beta-3",
  "term_id": "GO:0036376",
  "gene": "UniProtKB:P54709"
}